{
  "term_id": "GO:0005247",
  "gene_symbol": "CLCN6",
  "gene": "UniProtKB:P51797",
  "gene_name": "H(+)_Cl(-) exchange transporter 6",
  "term_label": "voltage-gated chloride channel activity"
}